{
  "gene": "UniProtKB:Q8TCC3",
  "gene_name": "Large ribosomal subunit protein uL30m",
  "term_label": "Unknown biological process",
  "term_id": "UNKNOWN:0002",
  "gene_symbol": "MRPL30"
}